superior vena cava morphogenesis [GO:0060578] (biological process) Definition: The process in which the anatomical structure of superior vena cava generated and organized. The superior vena cava is a blood vessel that transports blood from the upper body to the heart. Sources: GOC:dph Relationships: is a type of GO:0048845